innate immune response-inhibiting signal transduction [GO:0002766] (biological process) Definition: The cascade of processes by which a signal interacts with a receptor, causing a change in the level or activity of a second messenger or other downstream target, and ultimately leading to inhibition of an innate immune response. References: PMID:15771571 Sources: GOC:add, ISBN:0781735149 Relationships: is a type of immune response-inhibiting signal transduction [GO:0002765]